{
  "term_id": "GO:0051539",
  "gene_symbol": "ISCA2",
  "gene_name": "Iron-sulfur cluster assembly 2 homolog, mitochondrial",
  "gene": "UniProtKB:Q86U28",
  "term_label": "4 iron, 4 sulfur cluster binding"
}